{
  "term_id": "GO:0043197",
  "gene": "UniProtKB:Q02410",
  "gene_symbol": "APBA1",
  "term_label": "dendritic spine",
  "gene_name": "Amyloid-beta A4 precursor protein-binding family A member 1"
}